{
  "term_label": "molecular function activator activity",
  "gene_name": "Inner centromere protein",
  "term_id": "GO:0140677",
  "gene": "UniProtKB:Q9NQS7",
  "gene_symbol": "INCENP"
}